{
  "gene_name": "G1_S-specific cyclin-D3",
  "term_label": "microtubule organizing center",
  "gene": "UniProtKB:P30281",
  "gene_symbol": "CCND3",
  "term_id": "GO:0005815"
}